{
  "gene_symbol": "GNB3",
  "term_label": "cytoplasm",
  "term_id": "GO:0005737",
  "gene_name": "Guanine nucleotide-binding protein G(I)_G(S)_G(T) subunit beta-3",
  "gene": "UniProtKB:P16520"
}